regulation of eIF2 alpha phosphorylation by heme [GO:0010999] (BP) Definition: Any process that modulates the rate, frequency, or extent of eIF2 alpha phosphorylation as a result of heme levels. Relationships: is_a regulation of protein phosphorylation [GO:0001932]; is a type of GO:0006446; is a type of regulation of cellular response to stress [GO:0080135]; regulates GO:0010998 Sources: GOC:BHF, GOC:dph, GOC:tb